{
  "gene_name": "Cytoplasmic protein NCK1",
  "gene": "UniProtKB:P16333",
  "term_label": "cytoplasm",
  "gene_symbol": "NCK1",
  "term_id": "GO:0005737"
}